{
  "term_id": "GO:0005615",
  "gene": "UniProtKB:P09172",
  "gene_symbol": "DBH",
  "gene_name": "Dopamine beta-hydroxylase",
  "term_label": "extracellular space"
}